{
  "term_id": "GO:0031012",
  "gene_name": "Otoconin-90",
  "term_label": "extracellular matrix",
  "gene": "UniProtKB:Q02509",
  "gene_symbol": "OC90"
}